{
  "gene_symbol": "STAU1",
  "term_label": "protein localization to synapse",
  "term_id": "GO:0035418",
  "gene": "UniProtKB:O95793",
  "gene_name": "Double-stranded RNA-binding protein Staufen homolog 1"
}